{
  "gene_name": "MAPK-interacting and spindle-stabilizing protein-like",
  "term_id": "UNKNOWN:0003",
  "gene": "UniProtKB:Q8NDC0",
  "term_label": "Unknown cellular component",
  "gene_symbol": "MAPK1IP1L"
}